{
  "term_label": "RNA polymerase II cis-regulatory region sequence-specific DNA binding",
  "gene": "UniProtKB:Q6ZMS7",
  "term_id": "GO:0000978",
  "gene_symbol": "ZNF783",
  "gene_name": "Zinc finger protein 783"
}